{
  "gene_symbol": "CCDC163",
  "term_id": "UNKNOWN:0003",
  "gene": "UniProtKB:A0A0D9SF12",
  "gene_name": "Transmembrane protein CCDC163",
  "term_label": "Unknown cellular component"
}